{
  "term_id": "UNKNOWN:0002",
  "gene_name": "Arylsulfatase F",
  "gene_symbol": "ARSF",
  "gene": "UniProtKB:P54793",
  "term_label": "Unknown biological process"
}